cellular response to angiotensin [GO:1904385] (biological process) References: PMID:22982863 Sources: GOC:TermGenie, GO_REF:0000071 Relationships: is a type of cellular response to peptide hormone stimulus [GO:0071375]; is a type of response to angiotensin [GO:1990776] Definition: Any process that results in a change in state or activity of a cell (in terms of movement, secretion, enzyme production, gene expression, etc.) as a result of an angiotensin stimulus. Angiotensin is any of three physiologically active peptides (angiotensin II, III, or IV) processed from angiotensinogen.